{
  "term_id": "GO:0005654",
  "gene_name": "Spindlin-2B",
  "gene_symbol": "SPIN2B",
  "term_label": "nucleoplasm",
  "gene": "UniProtKB:Q9BPZ2"
}